{
  "gene_name": "G antigen 2B_2C",
  "gene": "UniProtKB:Q13066",
  "term_id": "UNKNOWN:0003",
  "term_label": "Unknown cellular component",
  "gene_symbol": "GAGE2C"
}